{
  "term_id": "GO:0009897",
  "gene_symbol": "RS1",
  "gene": "UniProtKB:O15537",
  "gene_name": "Retinoschisin",
  "term_label": "external side of plasma membrane"
}